{
  "term_label": "Unknown biological process",
  "gene": "UniProtKB:Q9GZY1",
  "term_id": "UNKNOWN:0002",
  "gene_symbol": "PBOV1",
  "gene_name": "Prostate and breast cancer overexpressed gene 1 protein"
}